sirohydrochlorin ferrochelatase activity [GO:0051266] (molecular function) Relationships: is a type of GO:0004325 Sources: RHEA:24360 Also known as: siroheme synthase activity, sirohydrochlorin ferro-lyase activity, siroheme ferro-lyase (sirohydrochlorin-forming) Definition: Catalysis of the reaction: siroheme + 2 H+ = Fe(2+) + sirohydrochlorin.